{
  "gene_symbol": "GAGE4",
  "gene_name": "G antigen 4",
  "gene": "UniProtKB:P0DSO3",
  "term_id": "UNKNOWN:0003",
  "term_label": "Unknown cellular component"
}